{
  "term_id": "GO:0016052",
  "term_label": "carbohydrate catabolic process",
  "gene": "UniProtKB:Q7L5Y1",
  "gene_symbol": "ENOSF1",
  "gene_name": "Mitochondrial enolase superfamily member 1"
}